{
  "term_id": "GO:0008630",
  "term_label": "intrinsic apoptotic signaling pathway in response to DNA damage",
  "gene_name": "Bcl-2 homologous antagonist_killer",
  "gene": "UniProtKB:Q16611",
  "gene_symbol": "BAK1"
}